{
  "gene_name": "Spermatogenesis-associated protein 31D4",
  "term_id": "UNKNOWN:0001",
  "term_label": "Unknown molecular function",
  "gene": "UniProtKB:Q6ZUB0",
  "gene_symbol": "SPATA31D4"
}